{
  "gene_name": "Protein ripply2",
  "term_id": "GO:0005634",
  "gene": "UniProtKB:Q5TAB7",
  "gene_symbol": "RIPPLY2",
  "term_label": "nucleus"
}